metanephric renal vesicle formation [GO:0072093] (biological process) Relationships: is a type of renal vesicle formation [GO:0072033]; is part of metanephric renal vesicle morphogenesis [GO:0072283] Also known as: metanephros formation Sources: GOC:mtg_kidney_jan10 Regulation: positively regulated by GO:0072094 Definition: The developmental process pertaining to the initial formation of the metanephros.